{
  "term_label": "cytoplasm",
  "term_id": "GO:0005737",
  "gene": "UniProtKB:Q14094",
  "gene_symbol": "CCNI",
  "gene_name": "Cyclin-I"
}